{
  "gene_symbol": "OCA2",
  "term_label": "Unknown molecular function",
  "term_id": "UNKNOWN:0001",
  "gene_name": "P protein",
  "gene": "UniProtKB:Q04671"
}